eukaryotic elongation factor-2 kinase regulator activity [GO:0042556] (molecular function) Subtypes: eukaryotic elongation factor-2 kinase activator activity [GO:0042557] Also known as: eEF-2 kinase regulator Definition: Modulates the activity of the enzyme eukaryotic elongation factor-2 kinase. Relationships: is a type of protein kinase regulator activity [GO:0019887]; regulates GO:0004686 References: PMID:11904175 Sources: GOC:jl